3',4',5'-trimethylmyricetin 3-O-methyltransferase activity [GO:0102440] (molecular function) Definition: Catalysis of the reaction: 3',4',5'-O-trimethylmyricetin + S-adenosyl-L-methionine = 3,3',4',5'-O-tetramethylmyricetin + S-adenosyl-L-homocysteine. Relationships: is a type of methyltransferase activity [GO:0008168] Sources: RHEA:74771